{
  "gene_name": "NADH dehydrogenase [ubiquinone] 1 beta subcomplex subunit 5, mitochondrial",
  "term_label": "Unknown biological process",
  "gene": "UniProtKB:O43674",
  "term_id": "UNKNOWN:0002",
  "gene_symbol": "NDUFB5"
}